{
  "term_id": "GO:0003729",
  "gene": "UniProtKB:A6NNA2",
  "term_label": "mRNA binding",
  "gene_symbol": "SRRM3",
  "gene_name": "Serine_arginine repetitive matrix protein 3"
}